voltage-gated calcium channel activity involved in Purkinje myocyte cell action potential [GO:0086058] (molecular function) Relationships: is a type of voltage-gated calcium channel activity involved in cardiac muscle cell action potential [GO:0086007]; is part of GO:0086047 Definition: Enables the transmembrane transfer of a calcium ion by a voltage-gated channel across the plasma membrane of an Purkinje myocyte cell that contributes to the depolarization phase of an action potential. A voltage-gated channel is a channel whose open state is dependent on the voltage across the membrane in which it is embedded. Sources: GOC:BHF, GOC:mtg_cardiac_conduct_nov11